{
  "term_label": "cytosol",
  "gene_name": "Fructose-bisphosphate aldolase C",
  "gene": "UniProtKB:P09972",
  "term_id": "GO:0005829",
  "gene_symbol": "ALDOC"
}